{
  "gene_symbol": "ZNF491",
  "term_label": "regulation of transcription by RNA polymerase II",
  "gene": "UniProtKB:Q8N8L2",
  "term_id": "GO:0006357",
  "gene_name": "Zinc finger protein 491"
}